{
  "gene_symbol": "PALLD",
  "term_id": "GO:0007411",
  "term_label": "axon guidance",
  "gene": "UniProtKB:Q8WX93",
  "gene_name": "Palladin"
}